{
  "gene": "UniProtKB:Q96DT7",
  "term_label": "RNA polymerase II transcription regulatory region sequence-specific DNA binding",
  "gene_symbol": "ZBTB10",
  "term_id": "GO:0000977",
  "gene_name": "Zinc finger and BTB domain-containing protein 10"
}